hexon binding [GO:0031423] (molecular function) Definition: Binding to a hexon, the major protein component of the icosahedral capsid of an adenovirus. References: PMID:12915569 Sources: GOC:mah Relationships: is a type of protein binding [GO:0005515]